{
  "gene_symbol": "SNX30",
  "gene": "UniProtKB:Q5VWJ9",
  "gene_name": "Sorting nexin-30",
  "term_label": "protein transport",
  "term_id": "GO:0015031"
}